{
  "gene": "UniProtKB:A0A1W2PPW3",
  "term_label": "transcription factor TFIID complex",
  "gene_symbol": "TAF11L12",
  "gene_name": "TATA-box-binding protein-associated factor 11-like protein 12",
  "term_id": "GO:0005669"
}